{
  "gene": "UniProtKB:O94844",
  "gene_symbol": "RHOBTB1",
  "gene_name": "Rho-related BTB domain-containing protein 1",
  "term_id": "GO:0007165",
  "term_label": "signal transduction"
}